photoperiodism [GO:0009648] (biological process) Relationships: is a type of response to light stimulus [GO:0009416] Sources: GOC:jid, GOC:pj, ISBN:0582015952, ISBN:0697037754, ISBN:0709408862 Subtypes: GO:0009906, response to photoperiod, red light [GO:0009907], entrainment of circadian clock by photoperiod [GO:0043153], GO:0048571, short-day photoperiodism [GO:0048572], photoperiodism, flowering [GO:0048573] Definition: Any process that results in a change in state or activity of an organism (in terms of movement, secretion, enzyme production, gene expression, etc.) as a result of detection of, or exposure to, a period of light or dark of a given length, measured relative to a particular duration known as the 'critical day length'. The critical day length varies between species. Also known as: response to day length, response to night length, response to photoperiod